{
  "gene_name": "Pregnancy-specific beta-1-glycoprotein 7",
  "gene_symbol": "PSG7",
  "term_label": "Unknown cellular component",
  "gene": "UniProtKB:Q13046",
  "term_id": "UNKNOWN:0003"
}